{
  "gene_name": "Zinc finger protein 559",
  "term_id": "GO:0005634",
  "gene_symbol": "ZNF559",
  "term_label": "nucleus",
  "gene": "UniProtKB:Q9BR84"
}